BORC complex [GO:0099078] (cellular component) Definition: A protein complex that is involved in positioning of the lysosome within the cytoplasm and which is composed of BLOC1S1, BLOC1S2, BORCS5, BORCS6, BORCS7, BORCS8, KXD1 and SNAPIN. The BORC complex recruits ARL8 at the cytosolic face of lysosomes and couples them to microtubule plus-end-directed kinesin motors. Relationships: is a type of GO:0140535 References: PMID:25898167 Sources: GOC:dos, GOC:li